{
  "gene_name": "Kinesin-like protein KIF9",
  "term_label": "kinesin complex",
  "term_id": "GO:0005871",
  "gene": "UniProtKB:Q9HAQ2",
  "gene_symbol": "KIF9"
}